{
  "gene": "UniProtKB:Q15032",
  "gene_name": "R3H domain-containing protein 1",
  "gene_symbol": "R3HDM1",
  "term_id": "UNKNOWN:0003",
  "term_label": "Unknown cellular component"
}